{
  "term_label": "Unknown molecular function",
  "gene_name": "Reticulon-4",
  "term_id": "UNKNOWN:0001",
  "gene": "UniProtKB:Q9NQC3",
  "gene_symbol": "RTN4"
}